{
  "gene_symbol": "ARHGAP1",
  "gene_name": "Rho GTPase-activating protein 1",
  "term_id": "GO:0005096",
  "term_label": "GTPase activator activity",
  "gene": "UniProtKB:Q07960"
}